pH-gated calcium channel activity [GO:0160126] (MF) Also known as: pH-dependent calcium channel activity, pH-sensitive calcium channel activity Definition: A gated channel activity that enables the transmembrane transfer of a calcium ion by a channel that opens in response to a change in pH. Relationships: is a type of ligand-gated calcium channel activity [GO:0099604]; is a type of pH-gated monoatomic ion channel activity [GO:0160128] References: PMID:30930064, PMID:34767445